subthalamus development [GO:0021539] (biological process) Definition: The process whose specific outcome is the progression of the subthalamus over time, from its formation to the mature structure. The subthalamus is the anterior part of the diencephalon that lies between the thalamus, hypothalamus, and tegmentum of the mesencephalon, including subthalamic nucleus, zona incerta, the fields of Forel, and the nucleus of ansa lenticularis. Sources: GOC:cls, GOC:dgh, GOC:dph, GOC:jid, GO_REF:0000021 Relationships: is a type of GO:0048856; is part of diencephalon development [GO:0021536] Also known as: ventral thalamus development